questin monooxygenase (NADPH) activity [GO:0050246] (molecular function) Relationships: is a type of oxidoreductase activity, acting on paired donors, with incorporation or reduction of molecular oxygen, NAD(P)H as one donor, and incorporation of one atom of oxygen [GO:0016709] Definition: Catalysis of the reaction: H+ + NADPH + O2 + questin = demethylsulochrin + NADP+. Also known as: questin oxygenase activity, questin,NADPH:oxygen oxidoreductase (hydroxylating, anthraquinone-ring-opening) Sources: RHEA:10836